DMNT synthase activity [GO:0102171] (MF) Definition: Catalysis of the reaction: (3S,6E)-nerolidol + O2 + reduced [NADPH--hemoprotein reductase] = (3E)-4,8-dimethylnona-1,3,7-triene + but-3-en-2-one + H+ + 2 H2O + oxidized [NADPH--hemoprotein reductase]. Sources: RHEA:55424 Relationships: is a type of oxidoreductase activity, acting on paired donors, with incorporation or reduction of molecular oxygen, reduced flavin or flavoprotein as one donor, and incorporation of one atom of oxygen [GO:0016712]